fructosamine metabolic process [GO:0030389] (BP) Subtypes: fructosamine biosynthetic process [GO:0030391], fructosamine catabolic process [GO:0030392], fructoselysine metabolic process [GO:0030393] Sources: GOC:jl, ISBN:0192801023 Relationships: is a type of GO:0006040 Also known as: fructosamine metabolism Definition: The chemical reactions and pathways involving fructosamine, a fructose molecule containing an amino group in place of a hydroxyl group.